terephthalate 1,2-dioxygenase activity [GO:0018628] (molecular function) Relationships: is a type of oxidoreductase activity, acting on paired donors, with incorporation or reduction of molecular oxygen, NAD(P)H as one donor, and incorporation of two atoms of oxygen into one donor [GO:0016708] Definition: Catalysis of the reaction: H+ + NADH + O2 + terephthalate = (3S,4R)-3,4-dihydroxycyclohexa-1,5-diene-1,4-dicarboxylate + NAD+. Also known as: 1,4-dicarboxybenzoate 1,2-dioxygenase activity, benzene-1,4-dicarboxylate 1,2-dioxygenase activity, benzene-1,4-dicarboxylate,NADH:oxygen oxidoreductase (1,2-hydroxylating) Sources: EC:1.14.12.15, RHEA:10312